3'-hydroxy-N-methyl-(S)-coclaurine 4'-O-methyltransferase activity [GO:0030784] (molecular function) Sources: EC:2.1.1.116 Definition: Catalysis of the reaction: S-adenosyl-L-methionine + 3'-hydroxy-N-methyl-(S)-coclaurine = S-adenosyl-L-homocysteine + (S)-reticuline. Relationships: is a type of S-adenosylmethionine-dependent methyltransferase activity [GO:0008757] Also known as: S-adenosyl-L-methionine:3'-hydroxy-N-methyl-(S)-coclaurine 4'-O-methyltransferase activity